{
  "gene": "UniProtKB:P17706",
  "gene_name": "Tyrosine-protein phosphatase non-receptor type 2",
  "term_id": "GO:0046426",
  "term_label": "negative regulation of receptor signaling pathway via JAK-STAT",
  "gene_symbol": "PTPN2"
}